{
  "gene_name": "Phospholipase D2",
  "gene_symbol": "PLD2",
  "term_id": "GO:0031410",
  "term_label": "cytoplasmic vesicle",
  "gene": "UniProtKB:O14939"
}